{
  "gene_symbol": "ATP2B1",
  "term_label": "regulation of cytosolic calcium ion concentration",
  "gene": "UniProtKB:P20020",
  "term_id": "GO:0051480",
  "gene_name": "Plasma membrane calcium-transporting ATPase 1"
}